tricellular tight junction assembly [GO:1904274] (biological process) Definition: The aggregation, arrangement and bonding together of a set of components to form a tricellular tight junction. Also known as: tricellular tight junction formation References: PMID:22640933, PMID:25097825, PMID:4203962 Sources: GOC:TermGenie, GOC:mr, GO_REF:0000079 Relationships: is a type of tight junction assembly [GO:0120192]